{
  "gene_name": "Symplekin",
  "term_id": "UNKNOWN:0002",
  "term_label": "Unknown biological process",
  "gene": "UniProtKB:Q92797",
  "gene_symbol": "SYMPK"
}